{
  "gene": "UniProtKB:Q9UJN7",
  "gene_symbol": "ZNF391",
  "term_id": "GO:0005634",
  "gene_name": "Zinc finger protein 391",
  "term_label": "nucleus"
}